Atg8-family ligase activity [GO:0019776] (molecular function) Relationships: is a type of ubiquitin-like protein ligase activity [GO:0061659] Definition: Catalysis of the covalent attachment of the ubiquitin-like protein Atg8 family modifier to phosphatidylethanolamine or phosphatidylserine on a membrane. References: PMID:12826404 Also known as: APG8 ligase activity, Atg8-like ligase activity, Atg8 ligase activity